{
  "gene_symbol": "ATP6V0C",
  "gene_name": "V-type proton ATPase 16 kDa proteolipid subunit c",
  "gene": "UniProtKB:P27449",
  "term_label": "membrane",
  "term_id": "GO:0016020"
}